{
  "gene_symbol": "PIGF",
  "term_id": "GO:0051377",
  "gene_name": "Phosphatidylinositol-glycan biosynthesis class F protein",
  "term_label": "mannose-ethanolamine phosphotransferase activity",
  "gene": "UniProtKB:Q07326"
}